{
  "term_label": "nucleus",
  "gene": "UniProtKB:Q8IUM7",
  "term_id": "GO:0005634",
  "gene_symbol": "NPAS4",
  "gene_name": "Neuronal PAS domain-containing protein 4"
}